arachidonate 12(R)-lipoxygenase activity [GO:0106237] (molecular function) Relationships: is_a oxidoreductase activity, acting on single donors with incorporation of molecular oxygen, incorporation of two atoms of oxygen [GO:0016702] References: PMID:10100631, PMID:11256953 Sources: GOC:gap, RHEA:41336 Definition: Catalysis of the reaction: arachidonate + O2 = (5Z,8Z,10E,12R,14Z)-12-hydroperoxyicosa-5,8,10,14-tetraenoate.